{
  "term_label": "calmodulin binding",
  "gene_name": "Calcium_calmodulin-dependent protein kinase type IV",
  "term_id": "GO:0005516",
  "gene": "UniProtKB:Q16566",
  "gene_symbol": "CAMK4"
}